{
  "term_label": "plasma membrane",
  "term_id": "GO:0005886",
  "gene": "UniProtKB:Q9BYE9",
  "gene_name": "Cadherin-related family member 2",
  "gene_symbol": "CDHR2"
}